{
  "gene": "UniProtKB:Q8ND24",
  "gene_name": "RING finger protein 214",
  "gene_symbol": "RNF214",
  "term_id": "UNKNOWN:0002",
  "term_label": "Unknown biological process"
}